patched binding [GO:0005113] (molecular function) Relationships: is a type of signaling receptor binding [GO:0005102] References: PMID:11731473 Sources: GOC:ceb Also known as: ptc binding, patched ligand, ptc ligand Definition: Binding to a patched (ptc) protein, a receptor for hedgehog proteins.